release of sequestered calcium ion into cytosol by sarcoplasmic reticulum [GO:0014808] (biological process) Regulation: regulated by regulation of release of sequestered calcium ion into cytosol by sarcoplasmic reticulum [GO:0010880] Relationships: is a type of sarcoplasmic reticulum calcium ion transport [GO:0070296]; is a type of release of sequestered calcium ion into cytosol by endoplasmic reticulum [GO:1903514] Definition: The process in which the release of sequestered calcium ion by sarcoplasmic reticulum into cytosol occurs via calcium release channels. Also known as: release of sequestered calcium ion by sarcoplasmic reticulum into cytosol Sources: GOC:mtg_muscle